platelet dense granule membrane [GO:0031088] (cellular component) Relationships: is a type of secretory granule membrane [GO:0030667]; is part of platelet dense granule [GO:0042827] Sources: GOC:mah Definition: The lipid bilayer surrounding the platelet dense granule.